{
  "term_id": "GO:0042361",
  "gene": "UniProtKB:P98187",
  "gene_name": "Cytochrome P450 4F8",
  "term_label": "menaquinone catabolic process",
  "gene_symbol": "CYP4F8"
}